{
  "gene": "UniProtKB:O95793",
  "term_id": "GO:0098964",
  "term_label": "anterograde dendritic transport of messenger ribonucleoprotein complex",
  "gene_symbol": "STAU1",
  "gene_name": "Double-stranded RNA-binding protein Staufen homolog 1"
}